{
  "term_label": "ubiquitin-dependent endocytosis",
  "gene_name": "E3 ubiquitin-protein ligase NEURL3",
  "gene": "UniProtKB:Q96EH8",
  "term_id": "GO:0070086",
  "gene_symbol": "NEURL3"
}